kinetochore organization [GO:0051383] (biological process) Definition: A process that is carried out at the cellular level which results in the assembly, arrangement of constituent parts, or disassembly of the kinetochore, a multisubunit complex that is located at the centromeric region of DNA and provides an attachment point for the spindle microtubules. Subtypes: kinetochore assembly [GO:0051382], kinetochore disassembly [GO:0062096] Also known as: kinetochore organisation, kinetochore organization and biogenesis Relationships: is_a chromosome organization [GO:0051276] Sources: GOC:ai, GOC:dph, GOC:jl, GOC:mah